{
  "term_label": "Unknown cellular component",
  "gene_symbol": "STAC3",
  "gene": "UniProtKB:Q96MF2",
  "term_id": "UNKNOWN:0003",
  "gene_name": "SH3 and cysteine-rich domain-containing protein 3"
}